{
  "gene": "UniProtKB:Q9C030",
  "gene_symbol": "TRIM6",
  "term_label": "cytoplasm",
  "term_id": "GO:0005737",
  "gene_name": "Tripartite motif-containing protein 6"
}